{
  "term_label": "DNA-binding transcription factor activity, RNA polymerase II-specific",
  "gene_symbol": "FOXD4L1",
  "gene_name": "Forkhead box protein D4-like 1",
  "term_id": "GO:0000981",
  "gene": "UniProtKB:Q9NU39"
}